{
  "gene_symbol": "NRXN3",
  "gene_name": "Neurexin-3",
  "term_id": "GO:0048787",
  "gene": "UniProtKB:Q9Y4C0",
  "term_label": "presynaptic active zone membrane"
}